{
  "term_label": "canonical Wnt signaling pathway",
  "gene_symbol": "WNT10B",
  "gene_name": "Protein Wnt-10b",
  "term_id": "GO:0060070",
  "gene": "UniProtKB:O00744"
}